{
  "gene_symbol": "KCNAB3",
  "term_label": "alcohol dehydrogenase (NADP+) activity",
  "gene_name": "Voltage-gated potassium channel subunit beta-3",
  "gene": "UniProtKB:O43448",
  "term_id": "GO:0008106"
}